{
  "gene": "UniProtKB:Q9ULL4",
  "gene_symbol": "PLXNB3",
  "term_label": "plasma membrane",
  "gene_name": "Plexin-B3",
  "term_id": "GO:0005886"
}